2-acetamido-4-O-(2-amino-2-deoxy-beta-D-glucopyranosyl)-2-deoxy-D-glucose exo-beta-D-glucosaminidase activity [GO:0102277] (molecular function) Definition: Catalysis of the reaction: beta-D-glucosaminyl-(1->4)-N-acetyl-D-glucosamine + H2O = D-glucosamine + N-acetyl-D-glucosamine. Sources: RHEA:62164 Relationships: is a type of hydrolase activity, hydrolyzing O-glycosyl compounds [GO:0004553]